{
  "gene_symbol": "PET100",
  "gene": "UniProtKB:P0DJ07",
  "term_label": "mitochondrial inner membrane",
  "term_id": "GO:0005743",
  "gene_name": "Protein PET100 homolog, mitochondrial"
}